{
  "gene": "UniProtKB:Q5T4F4",
  "gene_name": "Protrudin",
  "term_label": "vesicle-mediated transport",
  "term_id": "GO:0016192",
  "gene_symbol": "ZFYVE27"
}